{
  "gene_name": "Fibroblast growth factor receptor 1",
  "term_label": "fibroblast growth factor binding",
  "gene_symbol": "FGFR1",
  "term_id": "GO:0017134",
  "gene": "UniProtKB:P11362"
}